{
  "gene": "UniProtKB:Q9BW92",
  "term_id": "UNKNOWN:0003",
  "gene_name": "Threonine--tRNA ligase, mitochondrial",
  "gene_symbol": "TARS2",
  "term_label": "Unknown cellular component"
}